{
  "term_label": "DNA-binding transcription factor activity, RNA polymerase II-specific",
  "gene": "UniProtKB:Q2M1K9",
  "term_id": "GO:0000981",
  "gene_symbol": "ZNF423",
  "gene_name": "Zinc finger protein 423"
}